{
  "gene": "UniProtKB:Q9NYZ2",
  "term_label": "ferrous iron transmembrane transporter activity",
  "term_id": "GO:0015093",
  "gene_name": "Mitoferrin-1",
  "gene_symbol": "SLC25A37"
}